{
  "term_label": "Unknown molecular function",
  "gene_symbol": "TAMALIN",
  "term_id": "UNKNOWN:0001",
  "gene_name": "Protein TAMALIN",
  "gene": "UniProtKB:Q7Z6J2"
}